{
  "term_id": "UNKNOWN:0002",
  "gene_name": "Enkurin domain-containing protein 1",
  "term_label": "Unknown biological process",
  "gene": "UniProtKB:Q9H0I2",
  "gene_symbol": "ENKD1"
}